mature conventional dendritic cell differentiation [GO:0097029] (biological process) References: PMID:15845453 Sources: GOC:BHF Relationships: is a type of myeloid leukocyte differentiation [GO:0002573]; is a type of dendritic cell differentiation [GO:0097028] Definition: The process in which antigen-activated dendritic cells acquire the specialized features of a mature conventional dendritic cell. Mature conventional dendritic cells upregulate the surface expression of MHC molecules, chemokine receptors and adhesion molecules, and increase the number of dendrites (cytoplasmic protrusions) in preparation for migration to lymphoid organs where they present antigen to T cells. Note: Note that immunologists typically use the word 'maturation' to refer to dendritic cells undergoing the process that GO describes as 'cell differentiation'.